{
  "term_label": "sodium ion transmembrane transport",
  "gene_symbol": "SLC6A17",
  "gene_name": "Sodium-dependent neutral amino acid transporter SLC6A17",
  "term_id": "GO:0035725",
  "gene": "UniProtKB:Q9H1V8"
}